cellular response to gamma radiation [GO:0071480] (biological process) Regulation: RO_0002211 by regulation of cellular response to gamma radiation [GO:1905843]; negatively regulated by GO:1905844; positively regulated by GO:1905845 Definition: Any process that results in a change in state or activity of a cell (in terms of movement, secretion, enzyme production, gene expression, etc.) as a result of a gamma radiation stimulus. Gamma radiation is a form of electromagnetic radiation (EMR) or light emission of a specific frequency produced from sub-atomic particle interaction, such as electron-positron annihilation and radioactive decay. Gamma rays are generally characterized as EMR having the highest frequency and energy, and also the shortest wavelength, within the electromagnetic radiation spectrum. Also known as: cellular response to gamma ray, cellular response to gamma-ray photon Sources: GOC:mah Relationships: is a type of response to gamma radiation [GO:0010332]; is a type of GO:0071479